artery vasodilation involved in baroreceptor response to increased systemic arterial blood pressure [GO:0001984] (biological process) Also known as: vasodilation of artery involved in baroreceptor response to increased systemic arterial blood pressure Relationships: is a type of vasodilation [GO:0042311]; is part of baroreceptor response to increased systemic arterial blood pressure [GO:0001983] Definition: An increase in the internal diameter of an artery, triggered by vasomotor suppression, during the chemoreceptor response to decreased blood pressure. Sources: ISBN:0721643949